succinate-semialdehyde dehydrogenase (NAD+) activity [GO:0004777] (molecular function) Definition: Catalysis of the reaction: succinate semialdehyde + NAD+ + H2O = succinate + NADH + H+. Sources: RHEA:13217 Relationships: is a type of GO:0009013 Also known as: succinate semialdehyde dehydrogenase activity, succinate-semialdehyde dehydrogenase activity, succinic semialdehyde dehydrogenase activity, succinate semialdehyde:NAD+ oxidoreductase activity, succinate-semialdehyde:NAD+ oxidoreductase activity, succinyl semialdehyde dehydrogenase activity